{
  "gene_symbol": "UQCC1",
  "term_id": "GO:0034551",
  "term_label": "mitochondrial respiratory chain complex III assembly",
  "gene": "UniProtKB:Q9NVA1",
  "gene_name": "Ubiquinol-cytochrome-c reductase complex assembly factor 1"
}